{
  "term_label": "cytoplasm",
  "gene_name": "E3 ubiquitin-protein ligase MIB1",
  "gene": "UniProtKB:Q86YT6",
  "term_id": "GO:0005737",
  "gene_symbol": "MIB1"
}